{
  "gene_name": "Radial spoke head protein 3 homolog",
  "gene_symbol": "RSPH3",
  "term_id": "UNKNOWN:0002",
  "term_label": "Unknown biological process",
  "gene": "UniProtKB:Q86UC2"
}